{
  "term_id": "GO:1902388",
  "term_label": "ceramide 1-phosphate transfer activity",
  "gene": "UniProtKB:Q9NZD2",
  "gene_symbol": "GLTP",
  "gene_name": "Glycolipid transfer protein"
}